protein localization to kinetochore involved in kinetochore assembly [GO:1903394] (BP) References: PMID:15369671 Sources: GOC:TermGenie, GO_REF:0000060 Definition: Any protein localization to kinetochore that is involved in kinetochore assembly. Also known as: protein localisation to kinetochore involved in kinetochore assembly, condensin localization to kinetochore involved in centromere and kinetochore complex maturation, condensin localization to kinetochore involved in centromere/kinetochore complex maturation, condensin localization to kinetochore involved in chromosome-kinetochore attachment, condensin localization to kinetochore involved in kinetochore assembly, protein localisation to kinetochore involved in centromere and kinetochore complex maturation, protein localisation to kinetochore involved in centromere/kinetochore complex maturation, protein localisation to kinetochore involved in chromosome-kinetochore attachment, protein localization to kinetochore involved in centromere and kinetochore complex maturation, protein localization to kinetochore involved in centromere/kinetochore complex maturation, protein localization to kinetochore involved in chromosome-kinetochore attachment, condensin localization to kinetochore involved in kinetochore formation, protein localisation to kinetochore involved in kinetochore formation, protein localization to kinetochore involved in kinetochore formation Relationships: is a type of protein localization to kinetochore [GO:0034501]; BFO_0000050 kinetochore assembly [GO:0051382]